{
  "term_label": "cytoplasm",
  "gene": "UniProtKB:P28330",
  "gene_symbol": "ACADL",
  "gene_name": "Long-chain specific acyl-CoA dehydrogenase, mitochondrial",
  "term_id": "GO:0005737"
}